8-oxoguanine deaminase activity [GO:0102127] (molecular function) Definition: Catalysis of the reaction: H+ + 7,8-dihydro-8-oxoguanine + H2O = 7,9-dihydro-1H-purine-2,6,8(3H)-trione + ammonium. Sources: EC:3.5.4.32, GOC:pz Relationships: is a type of hydrolase activity, acting on carbon-nitrogen (but not peptide) bonds, in cyclic amidines [GO:0016814]